{
  "term_label": "nucleus",
  "gene": "UniProtKB:A4D1E1",
  "gene_symbol": "ZNF804B",
  "term_id": "GO:0005634",
  "gene_name": "Zinc finger protein 804B"
}